{
  "gene": "UniProtKB:P09619",
  "term_id": "GO:0005019",
  "gene_symbol": "PDGFRB",
  "term_label": "platelet-derived growth factor beta-receptor activity",
  "gene_name": "Platelet-derived growth factor receptor beta"
}